{
  "gene": "UniProtKB:Q9P2T1",
  "term_id": "UNKNOWN:0003",
  "gene_symbol": "GMPR2",
  "gene_name": "GMP reductase 2",
  "term_label": "Unknown cellular component"
}